{
  "gene_name": "Dehydrodolichyl diphosphate synthase complex subunit NUS1",
  "gene_symbol": "NUS1",
  "gene": "UniProtKB:Q96E22",
  "term_id": "GO:1904423",
  "term_label": "dehydrodolichyl diphosphate synthase complex"
}